meiotic DNA double-strand break formation involved in meiotic gene conversion [GO:0010781] (biological process) Sources: GOC:dph, GOC:tb Relationships: is a type of GO:0042138; is part of GO:0006311 Definition: The cell cycle process in which double-strand breaks are generated at defined hotspots throughout the genome during meiosis I resulting in meiotic gene conversion. Meiotic gene conversion is the cell cycle process in which genetic information is transferred from one helix to another.